ecdysone metabolic process [GO:0008205] (biological process) Sources: ISBN:0198506732 Subtypes: ecdysone biosynthetic process [GO:0006697], ecdysone catabolic process [GO:0006708] Definition: The chemical reactions and pathways involving ecdysone, (22R)-2-beta,3-beta,14,22,25-pentahydroxycholest-7-en-6-one, an ecdysteroid found in insects. It is the inactive prohormone of the moulting hormone ecdysterone and may have intrinsic hormonal activity at other stages of insect development. Relationships: is a type of sterol metabolic process [GO:0016125]; is_a ecdysteroid metabolic process [GO:0045455]; is a type of secondary alcohol metabolic process [GO:1902652] Also known as: ecdysone metabolism